{
  "term_label": "Unknown cellular component",
  "gene": "UniProtKB:Q96CX6",
  "gene_name": "Leucine-rich repeat-containing protein 58",
  "term_id": "UNKNOWN:0003",
  "gene_symbol": "LRRC58"
}